{
  "term_label": "regulation of transcription by RNA polymerase II",
  "gene_symbol": "HNRNPK",
  "gene": "UniProtKB:P61978",
  "gene_name": "Heterogeneous nuclear ribonucleoprotein K",
  "term_id": "GO:0006357"
}